{
  "gene_symbol": "GRM5",
  "gene_name": "Metabotropic glutamate receptor 5",
  "term_id": "GO:0001640",
  "term_label": "adenylate cyclase inhibiting G protein-coupled glutamate receptor activity",
  "gene": "UniProtKB:P41594"
}